bBAF complex [GO:0140092] (cellular component) Relationships: is a type of SWI/SNF superfamily-type complex [GO:0070603] Also known as: brain-specific BAF complex, brain-specific SWI/SNF complex References: PMID:12368262, PMID:12620226, PMID:15525990, PMID:17640523, PMID:17920018, PMID:8804307, PMID:8895581 Sources: GOC:bhm Definition: A brain-specific SWI/SNF-type complex that contains eight or nine proteins, including both conserved (core) and nonconserved components; contains the ATPase product of either the SMARCA4/BAF190A/BRG1 gene, the mammalian ortholog of the yeast SNF2 gene, or the SMARCA2/BAF190B/BRM gene, the mammalian ortholog of the Drosophila brm (brahma) gene, or an ortholog of either of these genes. Compared to the neuron-specific nBAF complex (GO:0071565) it does not contain DPF1, DPF3 or SMARCC1 or their orthologs. May contain PB1/BAF180.